protein-cysteine S-acyltransferase activity [GO:0019707] (molecular function) Subtypes: GO:0019705, protein-cysteine S-palmitoyltransferase activity [GO:0019706], GO:0140439, protein-cysteine S-oleoyltransferase activity [GO:0140440], protein-cysteine S-arachidonoyltransferase activity [GO:0140441] Sources: GOC:ai, RHEA:63372 Definition: Catalysis of the transfer of an acyl group to a sulfur atom on the cysteine of a protein molecule. Relationships: is a type of S-acyltransferase activity [GO:0016417]; is a type of catalytic activity, acting on a protein [GO:0140096]